endonucleolytic cleavage in ITS1 to separate SSU-rRNA from 5.8S rRNA and LSU-rRNA from tricistronic rRNA transcript (SSU-rRNA, 5.8S rRNA, LSU-rRNA) [GO:0000447] (biological process) Also known as: endonucleolytic cleavage at A2 Relationships: is a type of endonucleolytic cleavage of tricistronic rRNA transcript (SSU-rRNA, 5.8S rRNA, LSU-rRNA) [GO:0000479]; is part of maturation of SSU-rRNA from tricistronic rRNA transcript (SSU-rRNA, 5.8S rRNA, LSU-rRNA) [GO:0000462]; is part of maturation of 5.8S rRNA from tricistronic rRNA transcript (SSU-rRNA, 5.8S rRNA, LSU-rRNA) [GO:0000466] Definition: Endonucleolytic cleavage between the SSU-rRNA and the 5.8S rRNA of an rRNA molecule originally produced as a tricistronic rRNA transcript that contained the Small SubUnit (SSU) rRNA, the 5.8S rRNA, and the Large SubUnit (LSU) rRNA, in that order, from 5' to 3' along the primary transcript. References: PMID:10690410 Sources: GOC:curators